{
  "gene_symbol": "GFRAL",
  "term_id": "GO:0043235",
  "gene": "UniProtKB:Q6UXV0",
  "term_label": "receptor complex",
  "gene_name": "GDNF family receptor alpha-like"
}